{
  "gene_name": "Activated RNA polymerase II transcriptional coactivator p15",
  "gene": "UniProtKB:P53999",
  "gene_symbol": "SUB1",
  "term_id": "GO:0005667",
  "term_label": "transcription regulator complex"
}